{
  "gene": "UniProtKB:Q9UKL3",
  "gene_name": "CASP8-associated protein 2",
  "gene_symbol": "CASP8AP2",
  "term_id": "GO:0016605",
  "term_label": "PML body"
}